establishment of protein localization to mitochondrial membrane [GO:0090151] (biological process) Definition: The directed movement of a protein to a specific location in the mitochondrial membrane. Also known as: establishment of protein localisation in mitochondrial membrane, establishment of protein localization in mitochondrial membrane Subtypes: protein insertion into mitochondrial membrane [GO:0051204], establishment of protein localization to mitochondrial membrane involved in mitochondrial fission [GO:0090152] Relationships: is a type of mitochondrial membrane organization [GO:0007006]; is a type of establishment of localization in cell [GO:0051649]; is a type of establishment of protein localization to mitochondrion [GO:0072655]; is_a GO:0090150 Sources: GOC:ascb_2009, GOC:dph, GOC:tb